{
  "gene_symbol": "CASS4",
  "term_id": "GO:0016477",
  "gene_name": "Cas scaffolding protein family member 4",
  "term_label": "cell migration",
  "gene": "UniProtKB:Q9NQ75"
}